{
  "gene_symbol": "C4orf17",
  "term_id": "UNKNOWN:0001",
  "gene_name": "Uncharacterized protein C4orf17",
  "term_label": "Unknown molecular function",
  "gene": "UniProtKB:Q53FE4"
}